negative regulation of brown fat cell differentiation [GO:1903444] (biological process) Definition: Any process that stops, prevents or reduces the frequency, rate or extent of brown fat cell differentiation. References: PMID:23977283 Sources: GOC:TermGenie, GO_REF:0000058 Also known as: down regulation of brown adipocyte cell differentiation, down regulation of brown adipocyte differentiation, down regulation of brown fat cell differentiation, down-regulation of brown adipocyte cell differentiation, down-regulation of brown adipocyte differentiation, down-regulation of brown fat cell differentiation, downregulation of brown adipocyte cell differentiation, downregulation of brown adipocyte differentiation, downregulation of brown fat cell differentiation, negative regulation of brown adipocyte cell differentiation, negative regulation of brown adipocyte differentiation, inhibition of brown adipocyte cell differentiation, inhibition of brown adipocyte differentiation, inhibition of brown fat cell differentiation Relationships: is a type of negative regulation of fat cell differentiation [GO:0045599]; is a type of regulation of brown fat cell differentiation [GO:0090335]; negatively regulates GO:0050873